{
  "term_id": "GO:0030864",
  "gene": "UniProtKB:O75083",
  "gene_name": "WD repeat-containing protein 1",
  "gene_symbol": "WDR1",
  "term_label": "cortical actin cytoskeleton"
}